larval midgut histolysis [GO:0035069] (biological process) Definition: The stage-specific break down of the larval midgut during Drosophila metamorphosis, to allow replacement of larval structures by tissues and structures that form the adult fly. Relationships: is a type of anatomical structure regression [GO:0060033]; is part of GO:0007552; is part of instar larval or pupal morphogenesis [GO:0048707] Also known as: larval midgut regression References: PMID:9409683 Sources: GOC:bf, GOC:dph, GOC:mtg_apoptosis